{
  "gene_name": "SH3 domain-containing YSC84-like protein 1",
  "term_id": "GO:1900027",
  "gene": "UniProtKB:Q96HL8",
  "term_label": "regulation of ruffle assembly",
  "gene_symbol": "SH3YL1"
}